{
  "gene_symbol": "TRBV28",
  "gene_name": "T cell receptor beta variable 28",
  "term_id": "UNKNOWN:0001",
  "term_label": "Unknown molecular function",
  "gene": "UniProtKB:A0A5B6"
}